{
  "gene_symbol": "SEC24A",
  "term_id": "GO:0000149",
  "term_label": "SNARE binding",
  "gene_name": "Protein transport protein Sec24A",
  "gene": "UniProtKB:O95486"
}